{
  "gene_symbol": "MED26",
  "term_label": "core mediator complex",
  "gene_name": "Mediator of RNA polymerase II transcription subunit 26",
  "gene": "UniProtKB:O95402",
  "term_id": "GO:0070847"
}